negative regulation of alpha-beta T cell activation [GO:0046636] (biological process) Sources: GOC:ai Definition: Any process that stops, prevents, or reduces the frequency, rate or extent of alpha-beta T cell activation. Also known as: down regulation of alpha-beta T cell activation, down-regulation of alpha-beta T cell activation, downregulation of alpha-beta T cell activation, negative regulation of alpha-beta T lymphocyte activation, negative regulation of alpha-beta T-cell activation, negative regulation of alpha-beta T-lymphocyte activation, inhibition of alpha-beta T cell activation Subtypes: negative regulation of alpha-beta T cell differentiation [GO:0046639], negative regulation of alpha-beta T cell proliferation [GO:0046642], negative regulation of NK T cell activation [GO:0051134], negative regulation of CD4-positive, alpha-beta T cell activation [GO:2000515], negative regulation of CD8-positive, alpha-beta T cell activation [GO:2001186] Relationships: is a type of regulation of alpha-beta T cell activation [GO:0046634]; is a type of negative regulation of T cell activation [GO:0050868]; negatively regulates GO:0046631